{
  "term_label": "guanyl-nucleotide exchange factor activity",
  "gene": "UniProtKB:Q6VN20",
  "gene_symbol": "RANBP10",
  "term_id": "GO:0005085",
  "gene_name": "Ran-binding protein 10"
}